{
  "gene_name": "Uncharacterized protein",
  "gene_symbol": "A0A804HIB5",
  "gene": "UniProtKB:A0A804HIB5",
  "term_label": "Unknown molecular function",
  "term_id": "UNKNOWN:0001"
}